{
  "gene_symbol": "MAB21L2",
  "term_label": "Unknown biological process",
  "gene_name": "Protein mab-21-like 2",
  "gene": "UniProtKB:Q9Y586",
  "term_id": "UNKNOWN:0002"
}